{
  "gene_symbol": "GNA15",
  "term_id": "UNKNOWN:0001",
  "gene": "UniProtKB:P30679",
  "term_label": "Unknown molecular function",
  "gene_name": "Guanine nucleotide-binding protein subunit alpha-15"
}